methanol metabolic process [GO:0015945] (biological process) Sources: GOC:go_curators, ISBN:0198506732 Relationships: is a type of GO:0034308 Also known as: methanol metabolism Definition: The chemical reactions and pathways involving methanol, CH3-OH, a colorless, flammable, mobile, poisonous liquid, widely used as a solvent. Subtypes: methanol oxidation [GO:0015946], methanogenesis, from methanol [GO:0019387], GO:0046169, methanol catabolic process [GO:0046170]